ubiquitin recycling [GO:0010992] (biological process) References: PMID:19410548 Sources: GOC:BHF, GOC:dph, GOC:tb Definition: Any process involved in the maintenance of an internal steady state of ubiquitin monomers and free ubiquitin chains at the level of the cell by recycling ubiquitin from proteasome-bound ubiquitinated intermediates. Also known as: regulation of ubiquitin homeostasis, ubiquitin homeostasis Relationships: is a type of GO:0019725